{
  "term_id": "UNKNOWN:0002",
  "gene_name": "Oxysterol-binding protein-related protein 3",
  "gene": "UniProtKB:Q9H4L5",
  "term_label": "Unknown biological process",
  "gene_symbol": "OSBPL3"
}